{
  "gene_name": "Zinc finger and SCAN domain-containing protein 26",
  "term_label": "Unknown cellular component",
  "gene": "UniProtKB:Q16670",
  "term_id": "UNKNOWN:0003",
  "gene_symbol": "ZSCAN26"
}